{
  "gene": "UniProtKB:Q8IZP9",
  "term_id": "GO:0004930",
  "term_label": "G protein-coupled receptor activity",
  "gene_name": "Adhesion G-protein coupled receptor G2",
  "gene_symbol": "ADGRG2"
}